{
  "gene_symbol": "DERL1",
  "gene_name": "Derlin-1",
  "term_id": "GO:0030968",
  "gene": "UniProtKB:Q9BUN8",
  "term_label": "endoplasmic reticulum unfolded protein response"
}